{
  "gene_symbol": "CBFA2T3",
  "gene_name": "Protein CBFA2T3",
  "term_id": "GO:0045892",
  "term_label": "negative regulation of DNA-templated transcription",
  "gene": "UniProtKB:O75081"
}